{
  "term_label": "DNA ligase (ATP) activity",
  "term_id": "GO:0003910",
  "gene_symbol": "LIG4",
  "gene": "UniProtKB:P49917",
  "gene_name": "DNA ligase 4"
}